urokinase plasminogen activator signaling pathway [GO:0038195] (biological process) Relationships: is a type of GO:0007166 References: PMID:9417082 Sources: GOC:gap Also known as: uPA signaling pathway Definition: The series of molecular signals initiated by urokinase plasminogen activator binding to its receptor on the surface of a target cell, and ending with the regulation of a downstream cellular process, e.g. transcription.